signal recognition particle receptor complex [GO:0005785] (cellular component) Sources: ISBN:0198506732 Relationships: is a type of membrane protein complex [GO:0098796]; is a type of endoplasmic reticulum protein-containing complex [GO:0140534]; is part of rough endoplasmic reticulum membrane [GO:0030867] Also known as: SR complex, docking protein complex Definition: A transmembrane heterodimeric protein located in the membrane of the rough endoplasmic reticulum. Both subunits contain GTPase domains with which signal recognition particle interacts. In the presence of GTP and SRP receptor, SRP is released from the ribosome-nascent chain complex.